positive regulation of amino acid transport [GO:0051957] (BP) Sources: GOC:ai Definition: Any process that activates, maintains or increases the frequency, rate or extent of the directed movement of amino acids into, out of or within a cell, or between cells, by means of some agent such as a transporter or pore. Subtypes: positive regulation of L-glutamate import across plasma membrane [GO:0002038], positive regulation of glutamate secretion [GO:0014049], GO:0014054, positive regulation of amino acid uptake involved in synaptic transmission [GO:0051943], positive regulation of D-aspartate import across plasma membrane [GO:0140217], positive regulation of glycine import across plasma membrane [GO:1900925], GO:1900928, GO:1900931, positive regulation of proline import across plasma membrane [GO:1902836], positive regulation of aspartate secretion [GO:1904450], positive regulation of glycine secretion, neurotransmission [GO:1904626], positive regulation of L-lysine import across plasma membrane [GO:1905010], positive regulation of L-leucine import across plasma membrane [GO:1905534], GO:1905589, positive regulation of L-methionine import across plasma membrane [GO:1905626], positive regulation of glutamine transport [GO:2000487] Relationships: is a type of positive regulation of amine transport [GO:0051954]; is a type of regulation of amino acid transport [GO:0051955]; positively regulates amino acid transport [GO:0006865] Also known as: positive regulation of amino acid transmembrane transport, up regulation of amino acid transport, up-regulation of amino acid transport, upregulation of amino acid transport, activation of amino acid transport, stimulation of amino acid transport